{
  "term_id": "UNKNOWN:0003",
  "gene": "UniProtKB:B2CW77",
  "gene_symbol": "KLLN",
  "term_label": "Unknown cellular component",
  "gene_name": "Killin"
}